mammary gland alveolus development [GO:0060749] (biological process) Sources: GOC:dph Definition: The progression of the mammary gland alveolus over time, from its formation to its mature state. The mammary gland alveolus is a sac-like structure that is found in the mature gland. Relationships: is a type of anatomical structure development [GO:0048856]; BFO_0000050 mammary gland lobule development [GO:0061377]